{
  "gene": "UniProtKB:P25445",
  "gene_name": "Tumor necrosis factor receptor superfamily member 6",
  "term_label": "membrane raft",
  "term_id": "GO:0045121",
  "gene_symbol": "FAS"
}